{
  "gene": "UniProtKB:Q6VB84",
  "gene_name": "Forkhead box protein D4-like 3",
  "term_label": "Unknown cellular component",
  "gene_symbol": "FOXD4L3",
  "term_id": "UNKNOWN:0003"
}